{
  "term_label": "synaptic transmission, cholinergic",
  "gene": "UniProtKB:Q05901",
  "gene_symbol": "CHRNB3",
  "gene_name": "Neuronal acetylcholine receptor subunit beta-3",
  "term_id": "GO:0007271"
}